{
  "term_id": "GO:0071013",
  "gene_symbol": "ISY1",
  "gene_name": "Pre-mRNA-splicing factor ISY1 homolog",
  "term_label": "catalytic step 2 spliceosome",
  "gene": "UniProtKB:Q9ULR0"
}